negative regulation of protein localization to mitotic spindle pole body [GO:1902543] (biological process) Relationships: is a type of negative regulation of protein localization to spindle pole body [GO:1902364]; is a type of GO:1902542; negatively regulates protein localization to mitotic spindle pole body [GO:1902440] Also known as: down regulation of protein localisation to mitotic spindle pole body, down regulation of protein localization to mitotic spindle pole body, down-regulation of protein localisation in mitotic spindle pole body, down-regulation of protein localisation to mitotic spindle pole body, down-regulation of protein localization to mitotic spindle pole body, downregulation of protein localisation to mitotic spindle pole body, downregulation of protein localization to mitotic spindle pole body, negative regulation of protein localisation to mitotic spindle pole body, inhibition of protein localisation to mitotic spindle pole body, inhibition of protein localization to mitotic spindle pole body References: PMID:22809626 Sources: GOC:TermGenie Definition: Any process that stops, prevents or reduces the frequency, rate or extent of protein localization to mitotic spindle pole body.